{
  "gene": "UniProtKB:Q9UNA0",
  "gene_symbol": "ADAMTS5",
  "term_id": "GO:0030198",
  "term_label": "extracellular matrix organization",
  "gene_name": "A disintegrin and metalloproteinase with thrombospondin motifs 5"
}